{
  "gene": "UniProtKB:Q16581",
  "term_label": "plasma membrane",
  "gene_symbol": "C3AR1",
  "term_id": "GO:0005886",
  "gene_name": "C3a anaphylatoxin chemotactic receptor"
}